{
  "term_label": "Unknown cellular component",
  "term_id": "UNKNOWN:0003",
  "gene_name": "Acyl-CoA-binding domain-containing protein 7",
  "gene_symbol": "ACBD7",
  "gene": "UniProtKB:Q8N6N7"
}